triglyceride acyl-chain remodeling [GO:0036153] (biological process) Relationships: is a type of triglyceride metabolic process [GO:0006641]; is a type of acylglycerol acyl-chain remodeling [GO:0036155] References: PMID:15364929 Sources: GOC:mw Also known as: triacylglycerol acyl-chain remodeling, triglyceride acyl-chain remodelling Definition: Remodeling the acyl chains of triacylglycerol, through sequential deacylation and re-acylation reactions, to generate triacylglycerol containing different types of fatty acid acyl chains.